{
  "term_id": "UNKNOWN:0003",
  "gene_name": "Suppressor of cytokine signaling 3",
  "term_label": "Unknown cellular component",
  "gene_symbol": "SOCS3",
  "gene": "UniProtKB:O14543"
}